positive regulation of FACT complex assembly [GO:1905646] (biological process) Also known as: positive regulation of FACT complex formation, positive regulation of Facilitates chromatin transcription complex assembly, positive regulation of Facilitates chromatin transcription complex formation, up regulation of FACT complex assembly, up regulation of FACT complex formation, up regulation of Facilitates chromatin transcription complex assembly, up regulation of Facilitates chromatin transcription complex formation, up-regulation of FACT complex assembly, up-regulation of FACT complex formation, up-regulation of Facilitates chromatin transcription complex assembly, up-regulation of Facilitates chromatin transcription complex formation, upregulation of FACT complex assembly, upregulation of FACT complex formation, upregulation of Facilitates chromatin transcription complex assembly, upregulation of Facilitates chromatin transcription complex formation, activation of FACT complex assembly, activation of FACT complex formation, activation of Facilitates chromatin transcription complex assembly, activation of Facilitates chromatin transcription complex formation References: PMID:20889714 Sources: GOC:TermGenie, GO_REF:0000058 Definition: Any process that activates or increases the frequency, rate or extent of FACT complex assembly. Relationships: is a type of positive regulation of protein-containing complex assembly [GO:0031334]; is_a regulation of FACT complex assembly [GO:1905644]; positively regulates FACT complex assembly [GO:1905635]